{
  "gene": "UniProtKB:Q86XE5",
  "term_id": "GO:0005739",
  "gene_symbol": "HOGA1",
  "gene_name": "4-hydroxy-2-oxoglutarate aldolase, mitochondrial",
  "term_label": "mitochondrion"
}